negative regulation of synaptic vesicle lumen acidification [GO:1901547] (biological process) Also known as: down regulation of synaptic vesicle lumen acidification, down regulation of synaptic vesicle lumen pH reduction, down-regulation of synaptic vesicle lumen acidification, down-regulation of synaptic vesicle lumen pH reduction, downregulation of synaptic vesicle lumen acidification, downregulation of synaptic vesicle lumen pH reduction, negative regulation of proton loading, negative regulation of synaptic vesicle lumen pH reduction, inhibition of synaptic vesicle lumen acidification, inhibition of synaptic vesicle lumen pH reduction Sources: GOC:TermGenie Definition: Any process that stops, prevents or reduces the frequency, rate or extent of synaptic vesicle lumen acidification. Relationships: is a type of negative regulation of developmental process [GO:0051093]; is a type of regulation of synaptic vesicle lumen acidification [GO:1901546]; is a type of negative regulation of cation transmembrane transport [GO:1904063]; negatively regulates synaptic vesicle lumen acidification [GO:0097401]